{
  "term_label": "Unknown molecular function",
  "term_id": "UNKNOWN:0001",
  "gene_name": "Transcriptional regulator QRICH1",
  "gene": "UniProtKB:Q2TAL8",
  "gene_symbol": "QRICH1"
}